{
  "term_id": "GO:0003723",
  "gene_symbol": "RBM18",
  "gene": "UniProtKB:Q96H35",
  "gene_name": "Probable RNA-binding protein 18",
  "term_label": "RNA binding"
}